{
  "term_label": "type 3 melanocortin receptor binding",
  "term_id": "GO:0031781",
  "gene": "UniProtKB:Q8TCY5",
  "gene_name": "Melanocortin-2 receptor accessory protein",
  "gene_symbol": "MRAP"
}